6-hydroxypseudooxynicotine dehydrogenase activity [GO:0034909] (molecular function) Definition: Catalysis of the reaction: 6-hydroxypseudooxynicotine + H2O + OH- = 6-hydroxy-3-succinoylpyridine + 4 H+ + 4 e- + methylamine. Sources: UM-BBD_reactionID:r1441 Relationships: is a type of oxidoreductase activity, acting on the CH-NH group of donors [GO:0016645]